{
  "gene_symbol": "DYNC2I2",
  "term_id": "GO:0045504",
  "term_label": "dynein heavy chain binding",
  "gene": "UniProtKB:Q96EX3",
  "gene_name": "Cytoplasmic dynein 2 intermediate chain 2"
}